macronucleus organization [GO:0032124] (biological process) Definition: A process that is carried out at the cellular level which results in the assembly, arrangement of constituent parts, or disassembly of the macronucleus. References: PMID:10503190 Sources: GOC:dph, GOC:jl, GOC:mah Also known as: macronuclear organization, macronucleus organisation, macronuclear organization and biogenesis Relationships: is a type of nucleus organization [GO:0006997]